{
  "gene": "UniProtKB:Q9NW61",
  "gene_name": "Pleckstrin homology domain-containing family J member 1",
  "term_id": "UNKNOWN:0001",
  "term_label": "Unknown molecular function",
  "gene_symbol": "PLEKHJ1"
}